{
  "term_label": "potassium ion import across plasma membrane",
  "term_id": "GO:1990573",
  "gene_symbol": "SLC12A4",
  "gene": "UniProtKB:Q9UP95",
  "gene_name": "Solute carrier family 12 member 4"
}